{
  "gene_symbol": "UNC93B1",
  "gene": "UniProtKB:Q9H1C4",
  "term_id": "GO:0005768",
  "term_label": "endosome",
  "gene_name": "Protein unc-93 homolog B1"
}